oenocyte development [GO:0007438] (biological process) Definition: The process whose specific outcome is the progression of the oenocyte over time, from its formation to the mature structure. The oenocytes are large secretory cells found in clusters underlying the epidermis of larval abdominal segments. Relationships: is a type of GO:0048468; is part of oenocyte differentiation [GO:0001742] References: PMID:11171397 Sources: GOC:bf